adenosylhomocysteine nucleosidase activity [GO:0008782] (molecular function) Also known as: S-adenosylhomocysteine hydrolase activity, 5'-methyladenosine nucleosidase activity, AdoHcy/MTA nucleosidase activity, S-adenosyl-L-homocysteine homocysteinylribohydrolase activity, S-adenosylhomocysteine nucleosidase activity, S-adenosylhomocysteine/5'-methylthioadenosine nucleosidase activity Relationships: is a type of GO:0016799 Definition: Catalysis of the reaction: S-adenosyl-L-homocysteine + H2O = adenine + S-D-ribosyl-L-homocysteine. Sources: EC:3.2.2.9